plasmodesmatal endoplasmic reticulum [GO:0009511] (cellular component) Also known as: plasmodesmatal ER Relationships: is a type of endoplasmic reticulum [GO:0005783]; is part of plasmodesmatal desmotubule [GO:0009510] Definition: Endoplasmic reticulum found in plasmodesmata, junctions connecting the cytoplasm of adjacent plant cells. References: PMID:29880547 Sources: GOC:ai